subcortical maternal complex [GO:0106333] (cellular component) Definition: Comprised of at least NLRP5, OOEP, TLE6, and KHDC3/KHDC3L with evidence of additional SCMC-associated proteins that interact with one or multiple members of the core complex. Relationships: is a type of GO:0032991 References: PMID:18804437, PMID:28992324 Also known as: SCMC